{
  "gene": "UniProtKB:Q08629",
  "term_label": "calcium ion binding",
  "gene_symbol": "SPOCK1",
  "term_id": "GO:0005509",
  "gene_name": "Testican-1"
}